embryonic pelvic fin morphogenesis [GO:0035119] (biological process) Relationships: is a type of embryonic appendage morphogenesis [GO:0035113]; is a type of pelvic fin morphogenesis [GO:0035139] Sources: GOC:dgh Definition: The process, occurring in the embryo, by which the anatomical structures of the pelvic fin are generated and organized. The pelvic fins are bilaterally paired fins mounted in a ventral-lateral position on most fish. These fins are used primarily for lateral mobility and propulsion.